{
  "gene": "UniProtKB:P14672",
  "term_label": "perinuclear region of cytoplasm",
  "gene_symbol": "SLC2A4",
  "term_id": "GO:0048471",
  "gene_name": "Solute carrier family 2, facilitated glucose transporter member 4"
}